{
  "gene_name": "Major vault protein",
  "gene_symbol": "MVP",
  "term_id": "GO:0005634",
  "term_label": "nucleus",
  "gene": "UniProtKB:Q14764"
}